{
  "gene_name": "Cytotoxic T-lymphocyte protein 4",
  "gene": "UniProtKB:P16410",
  "term_id": "UNKNOWN:0001",
  "gene_symbol": "CTLA4",
  "term_label": "Unknown molecular function"
}